{
  "term_id": "GO:0008033",
  "gene_symbol": "TRMT1L",
  "gene_name": "TRMT1-like protein",
  "gene": "UniProtKB:Q7Z2T5",
  "term_label": "tRNA processing"
}